{
  "gene": "UniProtKB:P46778",
  "term_label": "cytosolic large ribosomal subunit",
  "term_id": "GO:0022625",
  "gene_name": "Large ribosomal subunit protein eL21",
  "gene_symbol": "RPL21"
}